{
  "term_id": "GO:0043325",
  "term_label": "phosphatidylinositol-3,4-bisphosphate binding",
  "gene_symbol": "ZFYVE1",
  "gene_name": "Zinc finger FYVE domain-containing protein 1",
  "gene": "UniProtKB:Q9HBF4"
}